{
  "term_label": "basement membrane",
  "term_id": "GO:0005604",
  "gene": "UniProtKB:P55268",
  "gene_symbol": "LAMB2",
  "gene_name": "Laminin subunit beta-2"
}